regulation of myotube differentiation [GO:0010830] (biological process) Sources: GOC:dph, GOC:tb Relationships: is_a GO:0051153; regulates myotube differentiation [GO:0014902] Definition: Any process that modulates the frequency, rate or extent of myotube differentiation. Myotube differentiation is the process in which a relatively unspecialized cell acquires specialized features of a myotube cell. Myotubes are multinucleated cells that are formed when proliferating myoblasts exit the cell cycle, differentiate and fuse. Subtypes: positive regulation of myotube differentiation [GO:0010831], negative regulation of myotube differentiation [GO:0010832], regulation of skeletal muscle fiber development [GO:0048742], regulation of skeletal muscle fiber differentiation [GO:1902809]